glutarate dioxygenase activity [GO:0106343] (molecular function) Relationships: is a type of 2-oxoglutarate-dependent dioxygenase activity [GO:0016706] References: PMID:30498244 Sources: RHEA:13821 Definition: Catalysis of the reaction glutarate + 2-oxoglutarate + O2 = (S)-2-hydroxyglutarate + succinate + CO2.